regulation of response to DNA damage checkpoint signaling [GO:1902153] (biological process) Subtypes: positive regulation of response to DNA damage checkpoint signaling [GO:1902154], regulation of response to G1 DNA damage checkpoint signaling [GO:1902155], GO:1902157 Also known as: regulation of DNA damage checkpoint effector process, regulation of response to signal involved in DNA damage checkpoint Relationships: is a type of regulation of response to DNA integrity checkpoint signaling [GO:1902151]; regulates response to DNA damage checkpoint signaling [GO:0072423] Definition: Any process that modulates the frequency, rate or extent of response to DNA damage checkpoint signaling. Sources: GOC:TermGenie, GOC:mtg_cell_cycle